immune effector process [GO:0002252] (biological process) Definition: Any process of the immune system that executes a component of an immune response. An effector immune process takes place after its activation. Subtypes: cell activation involved in immune response [GO:0002263], granuloma formation [GO:0002432], immune response-regulating cell surface receptor signaling pathway involved in phagocytosis [GO:0002433], immune complex clearance [GO:0002434], leukocyte mediated immunity [GO:0002443], leukocyte migration involved in immune response [GO:0002522], respiratory burst involved in defense response [GO:0002679], complement activation [GO:0006956], opsonization [GO:0008228], induced systemic resistance, jasmonic acid mediated signaling pathway [GO:0009864], induced systemic resistance, ethylene mediated signaling pathway [GO:0009866], encapsulation of foreign target [GO:0035010], leukocyte degranulation [GO:0043299] Sources: GOC:add, GO_REF:0000022, ISBN:0781735149 Regulation: regulated by regulation of immune effector process [GO:0002697]; negatively regulated by negative regulation of immune effector process [GO:0002698]; positively regulated by GO:0002699 Relationships: is a type of GO:0002376